{
  "term_label": "Unknown cellular component",
  "gene_name": "Interleukin-32",
  "term_id": "UNKNOWN:0003",
  "gene_symbol": "IL32",
  "gene": "UniProtKB:P24001"
}